{
  "gene": "UniProtKB:Q58FF3",
  "gene_name": "Putative endoplasmin-like protein",
  "term_label": "unfolded protein binding",
  "gene_symbol": "HSP90B2P",
  "term_id": "GO:0051082"
}